{
  "gene_name": "G-protein-signaling modulator 1",
  "gene": "UniProtKB:Q86YR5",
  "term_label": "GDP-dissociation inhibitor activity",
  "term_id": "GO:0005092",
  "gene_symbol": "GPSM1"
}